syncytium formation by plasma membrane fusion [GO:0000768] (biological process) Also known as: cell fusion Sources: GOC:mtg_muscle, GOC:tb Regulation: RO_0002212 by negative regulation of syncytium formation by plasma membrane fusion [GO:0034242]; regulated by regulation of syncytium formation by plasma membrane fusion [GO:0060142]; positively regulated by positive regulation of syncytium formation by plasma membrane fusion [GO:0060143] Subtypes: myoblast fusion [GO:0007520], macrophage fusion [GO:0034238], osteoclast fusion [GO:0072675] Definition: The formation of a syncytium, a mass of cytoplasm containing several nuclei enclosed within a single plasma membrane, by the fusion of the plasma membranes of two or more individual cells. Relationships: is a type of syncytium formation [GO:0006949]; is a type of cell-cell fusion [GO:0140253]